{
  "term_id": "GO:0005634",
  "term_label": "nucleus",
  "gene_name": "SWI_SNF-related matrix-associated actin-dependent regulator of chromatin subfamily A containing DEAD_H box 1",
  "gene_symbol": "SMARCAD1",
  "gene": "UniProtKB:Q9H4L7"
}